chlorosome [GO:0046858] (cellular component) References: PMID:14729689, PMID:15298919 Sources: ISBN:0198506732 Relationships: is_a intracellular membraneless organelle [GO:0043232] Definition: A large enclosure of aggregated pigment, typically bacteriochlorophyll c (BChl c), that acts as a light-harvesting antenna structure and is characteristic of green photosynthetic bacteria (e.g. Chlorobiaceae). The BChl aggregates are organized into lamellar elements by pigment-pigment rather than pigment-protein interactions. Chlorosomes also contain BChl a, carotenoids, quinones, lipids, and proteins, and are attached to the cytoplasmic membrane via a BChl a-containing protein baseplate.